main body follicle cell migration [GO:0060270] (biological process) Relationships: is a type of follicle cell of egg chamber migration [GO:0007297] Sources: GOC:dph Definition: The ovarian follicle cell migration process in which follicle cells migrate posteriorly to form a columnar epithelium over the oocyte.